peptidyl-tyrosine sulfation [GO:0006478] (biological process) Definition: The sulfation of peptidyl-tyrosine residues to form peptidyl-O4'-sulfo-L-tyrosine. Sources: RESID:AA0172 Also known as: peptidyl-tyrosine sulphation Relationships: is a type of GO:0006477; is a type of peptidyl-tyrosine modification [GO:0018212]